{
  "gene_symbol": "P0DMU3",
  "gene": "UniProtKB:P0DMU3",
  "term_id": "UNKNOWN:0001",
  "term_label": "Unknown molecular function",
  "gene_name": "FAM231A_C-like protein LOC102723383"
}